1,6-anhydro-N-acetyl-beta-muramic acid catabolic process [GO:0097175] (biological process) Relationships: is a type of monocarboxylic acid catabolic process [GO:0072329] References: PMID:15901686 Sources: GOC:yaf Also known as: 1,6-anhydro-N-acetyl-beta-muramate breakdown, 1,6-anhydro-N-acetyl-beta-muramate catabolic process, 1,6-anhydro-N-acetyl-beta-muramate catabolism, 1,6-anhydro-N-acetyl-beta-muramate degradation, 1,6-anhydro-N-acetyl-beta-muramic acid breakdown, 1,6-anhydro-N-acetyl-beta-muramic acid catabolism, 1,6-anhydro-N-acetyl-beta-muramic acid degradation, 1,6-anhydro-N-acetylmuramate breakdown, 1,6-anhydro-N-acetylmuramate catabolic process, 1,6-anhydro-N-acetylmuramate catabolism, 1,6-anhydro-N-acetylmuramate degradation, 1,6-anhydro-N-acetylmuramic acid breakdown, 1,6-anhydro-N-acetylmuramic acid catabolic process, 1,6-anhydro-N-acetylmuramic acid catabolism, 1,6-anhydro-N-acetylmuramic acid degradation Definition: The chemical reactions and pathways resulting in the breakdown of 1,6-anhydro-N-acetylmuramic acid, the 1,6-anhydro-derivative of N-acetyl-beta-muramic acid.